response to L-phenylalanine derivative [GO:1904386] (biological process) Definition: Any process that results in a change in state or activity of a cell or an organism (in terms of movement, secretion, enzyme production, gene expression, etc.) as a result of a L-phenylalanine derivative stimulus. Subtypes: response to thyroxine [GO:0097068], cellular response to L-phenylalanine derivative [GO:1904387], response to L-dopa [GO:1904473] References: PMID:12112407 Sources: GOC:TermGenie, GO_REF:0000071 Relationships: is a type of response to nitrogen compound [GO:1901698]